{
  "term_id": "GO:0098839",
  "gene_name": "Glutamate receptor ionotropic, delta-1",
  "gene": "UniProtKB:Q9ULK0",
  "term_label": "postsynaptic density membrane",
  "gene_symbol": "GRID1"
}